{
  "gene_symbol": "CWF19L2",
  "gene_name": "CWF19-like protein 2",
  "term_label": "Unknown molecular function",
  "gene": "UniProtKB:Q2TBE0",
  "term_id": "UNKNOWN:0001"
}